{
  "gene_name": "Plastin-1",
  "gene": "UniProtKB:Q14651",
  "gene_symbol": "PLS1",
  "term_id": "GO:0051015",
  "term_label": "actin filament binding"
}